{
  "term_id": "GO:0009311",
  "gene_symbol": "ST8SIA5",
  "gene_name": "Alpha-2,8-sialyltransferase 8E",
  "term_label": "oligosaccharide metabolic process",
  "gene": "UniProtKB:O15466"
}